{
  "term_id": "GO:0005634",
  "gene_symbol": "SP4",
  "gene_name": "Transcription factor Sp4",
  "gene": "UniProtKB:Q02446",
  "term_label": "nucleus"
}